{
  "gene_symbol": "OR9A4",
  "term_id": "UNKNOWN:0002",
  "gene_name": "Olfactory receptor 9A4",
  "term_label": "Unknown biological process",
  "gene": "UniProtKB:Q8NGU2"
}